{
  "gene_symbol": "CD2",
  "term_label": "signaling receptor binding",
  "gene_name": "T-cell surface antigen CD2",
  "term_id": "GO:0005102",
  "gene": "UniProtKB:P06729"
}